{
  "term_label": "centriole",
  "gene_name": "POC1 centriolar protein homolog A",
  "gene": "UniProtKB:Q8NBT0",
  "gene_symbol": "POC1A",
  "term_id": "GO:0005814"
}